positive regulation of chromosome condensation [GO:1905821] (biological process) Subtypes: positive regulation of mitotic chromosome condensation [GO:1903380] References: PMID:17268547 Sources: GOC:TermGenie, GOC:bhm, GO_REF:0000058 Definition: Any process that activates or increases the frequency, rate or extent of chromosome condensation. Relationships: is a type of regulation of chromosome condensation [GO:0060623]; is a type of GO:2001252; positively regulates chromosome condensation [GO:0030261] Also known as: positive regulation of eukaryotic chromosome condensation, positive regulation of nuclear chromosome condensation, up regulation of chromosome condensation, up regulation of eukaryotic chromosome condensation, up regulation of nuclear chromosome condensation, up-regulation of chromosome condensation, up-regulation of eukaryotic chromosome condensation, up-regulation of nuclear chromosome condensation, upregulation of chromosome condensation, upregulation of eukaryotic chromosome condensation, upregulation of nuclear chromosome condensation, activation of chromosome condensation, activation of eukaryotic chromosome condensation, activation of nuclear chromosome condensation